aldehyde oxidase activity [GO:0004031] (molecular function) Also known as: retinal oxidase activity, aldehyde:oxygen oxidoreductase activity, quinoline oxidase activity Relationships: is a type of oxidoreductase activity, acting on the aldehyde or oxo group of donors, oxygen as acceptor [GO:0016623] Subtypes: pyridoxal oxidase activity [GO:0004732], GO:0018488 Definition: Catalysis of the reaction: an aldehyde + H2O + O2 = a carboxylic acid + hydrogen peroxide. Sources: EC:1.2.3.1